{
  "gene": "UniProtKB:Q8NBF4",
  "term_id": "UNKNOWN:0001",
  "term_label": "Unknown molecular function",
  "gene_symbol": "Q8NBF4",
  "gene_name": "Putative uncharacterized protein FLJ33307"
}